17alpha-hydroxyprogesterone binding [GO:1903880] (molecular function) References: PMID:10802282 Sources: GOC:TermGenie, GOC:mr, GO_REF:0000067 Relationships: is a type of steroid binding [GO:0005496]; is a type of alcohol binding [GO:0043178] Definition: Binding to 17alpha-hydroxyprogesterone.